developmental growth involved in morphogenesis [GO:0060560] (biological process) Sources: GOC:dph Also known as: differential growth Relationships: is a type of developmental growth [GO:0048589]; is part of anatomical structure morphogenesis [GO:0009653] Subtypes: growth involved in heart morphogenesis [GO:0003241], axis elongation [GO:0003401], optic vesicle elongation [GO:0003405], growth plate cartilage chondrocyte growth [GO:0003430], unidimensional cell growth [GO:0009826], dorsal trunk growth, open tracheal system [GO:0035001], elongation of arista core [GO:0035015], elongation of arista lateral [GO:0035016], nephric duct elongation [GO:0035849], GO:0044181, GO:0048526, collateral sprouting [GO:0048668], sprouting of injured axon [GO:0048682], root hair elongation [GO:0048767], outer ear emergence [GO:0060186], GO:0060649, ureteric bud elongation [GO:0060677], primary ureteric bud growth [GO:0060682], prostate gland morphogenetic growth [GO:0060737], mammary duct terminal end bud growth [GO:0060763], bud dilation [GO:0061137], cell growth involved in Malpighian tubule morphogenesis [GO:0061335], ureteric bud invasion [GO:0072092], neuron projection extension [GO:1990138] Definition: The increase in size or mass of an anatomical structure that contributes to the structure attaining its shape.